{
  "term_label": "amino acid transmembrane transport",
  "gene_name": "Neutral amino acid transporter 9",
  "gene_symbol": "SLC38A9",
  "term_id": "GO:0003333",
  "gene": "UniProtKB:Q8NBW4"
}